spleen trabecula formation [GO:0060345] (biological process) Sources: GOC:dph Also known as: spleen trabeculation, spleen trabecula biogenesis Definition: The process of creating a trabecula in the spleen. A trabecula is a tissue element in the form of a small beam, strut or rod. Relationships: is a type of trabecula formation [GO:0060343]; is part of spleen development [GO:0048536]